{
  "term_id": "GO:0090575",
  "term_label": "RNA polymerase II transcription regulator complex",
  "gene_name": "Retinoic acid receptor alpha",
  "gene": "UniProtKB:P10276",
  "gene_symbol": "RARA"
}